{
  "term_id": "GO:0004175",
  "gene": "UniProtKB:P28072",
  "term_label": "endopeptidase activity",
  "gene_name": "Proteasome subunit beta type-6",
  "gene_symbol": "PSMB6"
}